{
  "term_label": "integrin binding",
  "gene": "UniProtKB:P26010",
  "term_id": "GO:0005178",
  "gene_symbol": "ITGB7",
  "gene_name": "Integrin beta-7"
}